{
  "term_id": "GO:0019901",
  "gene": "UniProtKB:P0DV79",
  "gene_symbol": "SPDYE18",
  "gene_name": "Speedy protein E18",
  "term_label": "protein kinase binding"
}